{
  "gene": "UniProtKB:P0C7W6",
  "gene_name": "Coiled-coil domain-containing protein 172",
  "gene_symbol": "CCDC172",
  "term_label": "Unknown molecular function",
  "term_id": "UNKNOWN:0001"
}